{
  "gene_name": "Nuclear pore complex-interacting protein family member B11",
  "gene": "UniProtKB:E5RHQ5",
  "term_label": "Unknown cellular component",
  "term_id": "UNKNOWN:0003",
  "gene_symbol": "NPIPB11"
}